{
  "term_id": "UNKNOWN:0001",
  "gene_symbol": "TUSC2",
  "gene_name": "Tumor suppressor candidate 2",
  "gene": "UniProtKB:O75896",
  "term_label": "Unknown molecular function"
}